{
  "term_label": "lipid droplet organization",
  "gene": "UniProtKB:Q9NP72",
  "gene_name": "Ras-related protein Rab-18",
  "gene_symbol": "RAB18",
  "term_id": "GO:0034389"
}